histone crotonyltransferase activity [GO:0140068] (molecular function) References: PMID:25818647 Definition: Catalysis of the reaction: crotonyl-CoA + histone = CoA + crotonyl-histone. Relationships: is a type of peptide crotonyltransferase activity [GO:0140064]; is a type of histone modifying activity [GO:0140993]